{
  "gene_symbol": "NAA80",
  "gene_name": "N-alpha-acetyltransferase 80",
  "term_id": "GO:1905502",
  "gene": "UniProtKB:Q93015",
  "term_label": "acetyl-CoA binding"
}